{
  "gene_symbol": "POTEJ",
  "gene_name": "POTE ankyrin domain family member J",
  "gene": "UniProtKB:P0CG39",
  "term_id": "GO:0045202",
  "term_label": "synapse"
}